response to 1-oleoyl-sn-glycerol 3-phosphate [GO:1904565] (biological process) Definition: Any process that results in a change in state or activity of a cell or an organism (in terms of movement, secretion, enzyme production, gene expression, etc.) as a result of a 1-oleoyl-sn-glycerol 3-phosphate stimulus. References: PMID:12139919 Sources: GOC:TermGenie, GO_REF:0000071 Also known as: response to 1-oleoyl lysophosphatidic acid, response to LPA, response to lysophosphatidic acid, response to oleoyl lysophosphatidic acid, response to oleoyl-L-alpha-lysophosphatidic acid Relationships: is a type of GO:0033993; is_a response to organophosphorus [GO:0046683]; is a type of GO:1901700 Subtypes: cellular response to 1-oleoyl-sn-glycerol 3-phosphate [GO:1904566]